{
  "gene": "UniProtKB:Q99727",
  "gene_name": "Metalloproteinase inhibitor 4",
  "term_label": "metalloendopeptidase inhibitor activity",
  "term_id": "GO:0008191",
  "gene_symbol": "TIMP4"
}